{
  "gene_name": "Transmembrane protein 178A",
  "term_label": "endoplasmic reticulum membrane",
  "term_id": "GO:0005789",
  "gene_symbol": "TMEM178A",
  "gene": "UniProtKB:Q8NBL3"
}